{
  "gene": "UniProtKB:Q9H4F1",
  "term_id": "GO:0001665",
  "term_label": "alpha-N-acetylgalactosaminide alpha-2,6-sialyltransferase activity",
  "gene_name": "Alpha-N-acetyl-neuraminyl-2,3-beta-galactosyl-1,3-N-acetyl-galactosaminide alpha-2,6-sialyltransferase",
  "gene_symbol": "ST6GALNAC4"
}